{
  "gene_symbol": "TEPSIN",
  "gene": "UniProtKB:Q96N21",
  "term_id": "UNKNOWN:0001",
  "term_label": "Unknown molecular function",
  "gene_name": "AP-4 complex accessory subunit Tepsin"
}